{
  "term_label": "ganglioside biosynthetic process",
  "gene": "UniProtKB:Q9H4F1",
  "term_id": "GO:0001574",
  "gene_name": "Alpha-N-acetyl-neuraminyl-2,3-beta-galactosyl-1,3-N-acetyl-galactosaminide alpha-2,6-sialyltransferase",
  "gene_symbol": "ST6GALNAC4"
}